{
  "gene_symbol": "APOM",
  "gene": "UniProtKB:O95445",
  "term_label": "lipid transporter activity",
  "gene_name": "Apolipoprotein M",
  "term_id": "GO:0005319"
}